{
  "term_label": "mitochondrial large ribosomal subunit",
  "gene": "UniProtKB:Q13405",
  "gene_name": "Large ribosomal subunit protein mL49",
  "term_id": "GO:0005762",
  "gene_symbol": "MRPL49"
}